negative regulation of catecholamine secretion [GO:0033604] (biological process) Also known as: down regulation of catecholamine secretion, down-regulation of catecholamine secretion, downregulation of catecholamine secretion, inhibition of catecholamine secretion Subtypes: negative regulation of norepinephrine secretion [GO:0010700], negative regulation of epinephrine secretion [GO:0032811], GO:0033602 Definition: Any process that stops, prevents, or reduces the frequency, rate or extent of the regulated release of a catecholamine. Relationships: is a type of GO:0050433; is a type of GO:0051953; is a type of negative regulation of secretion by cell [GO:1903531]; negatively regulates GO:0050432 Sources: GOC:mah